{
  "gene_symbol": "SRSF5",
  "term_id": "GO:0016607",
  "term_label": "nuclear speck",
  "gene": "UniProtKB:Q13243",
  "gene_name": "Serine_arginine-rich splicing factor 5"
}